{
  "term_id": "GO:0000139",
  "gene_name": "E3 ubiquitin-protein ligase HACE1",
  "term_label": "Golgi membrane",
  "gene_symbol": "HACE1",
  "gene": "UniProtKB:Q8IYU2"
}